carnitine transmembrane transporter activity [GO:0015226] (molecular function) Subtypes: GO:0005476, (R)-carnitine transmembrane transporter activity [GO:1901235] Definition: Enables the transfer of carnitine across a membrane. Carnitine is a compound that participates in the transfer of acyl groups across the inner mitochondrial membrane. Sources: GOC:ai Also known as: vitamin Bt transporter activity Relationships: is a type of quaternary ammonium group transmembrane transporter activity [GO:0015651]; is_a GO:0072349; is part of GO:1902603